 [RO:0002161]